{
  "gene_name": "SH2 domain-containing protein 4B",
  "term_label": "cytoplasm",
  "term_id": "GO:0005737",
  "gene_symbol": "SH2D4B",
  "gene": "UniProtKB:Q5SQS7"
}